{
  "gene_symbol": "ZC3HAV1L",
  "gene": "UniProtKB:Q96H79",
  "gene_name": "Zinc finger CCCH-type antiviral protein 1-like",
  "term_label": "Unknown biological process",
  "term_id": "UNKNOWN:0002"
}